positive regulation of telomere maintenance via semi-conservative replication [GO:0032215] (biological process) Definition: Any process that activates or increases the frequency, rate or extent of the semi-conservative replication of telomeric DNA. Sources: GOC:mah Also known as: up regulation of telomere maintenance via semi-conservative replication, up-regulation of telomere maintenance via semi-conservative replication, upregulation of telomere maintenance via semi-conservative replication, activation of telomere maintenance via semi-conservative replication, stimulation of telomere maintenance via semi-conservative replication Relationships: is a type of positive regulation of telomere maintenance [GO:0032206]; is_a regulation of telomere maintenance via semi-conservative replication [GO:0032213]; is a type of positive regulation of cell cycle process [GO:0090068]; positively regulates GO:0032201